{
  "gene_symbol": "RPGR",
  "term_label": "photoreceptor outer segment",
  "term_id": "GO:0001750",
  "gene": "UniProtKB:Q92834",
  "gene_name": "X-linked retinitis pigmentosa GTPase regulator"
}